{
  "term_id": "UNKNOWN:0002",
  "gene_symbol": "BTBD10",
  "gene": "UniProtKB:Q9BSF8",
  "term_label": "Unknown biological process",
  "gene_name": "BTB_POZ domain-containing protein 10"
}